{
  "term_label": "cell differentiation",
  "gene_name": "Mothers against decapentaplegic homolog 9",
  "gene": "UniProtKB:O15198",
  "term_id": "GO:0030154",
  "gene_symbol": "SMAD9"
}